{
  "term_id": "UNKNOWN:0002",
  "gene_name": "Beta-1-syntrophin",
  "gene": "UniProtKB:Q13884",
  "term_label": "Unknown biological process",
  "gene_symbol": "SNTB1"
}